(R)-2-methylmalate dehydratase activity [GO:0047508] (MF) Relationships: is_a hydro-lyase activity [GO:0016836] Also known as: (-)-citramalate hydro-lyase activity, (R)-2-methylmalate hydro-lyase (2-methylmaleate-forming), (R)-2-methylmalate hydro-lyase activity, citraconase activity, citraconate hydratase activity, citramalate hydro-lyase activity Definition: Catalysis of the reaction: (R)-citramalate = 2-methylmaleate + H2O. Sources: EC:4.2.1.35